venom-mediated perturbation of blood coagulation [GO:0044468] (biological process) Definition: A process in which an organism alters or subverts blood coagulation in another organism via the action of a venom. Relationships: is a type of venom-mediated perturbation of hemostasis [GO:0044483] Also known as: envenomation perturbing blood coagulation, envenomation resulting in modulation of blood coagulation in another organism, envenomation resulting in modulation of blood coagulation in other organism, envenomation resulting in perturbation of blood coagulation, envenomation resulting in regulation of blood coagulation in other organism Subtypes: venom-mediated blood coagulation [GO:0044469], venom-mediated suppression of blood coagulation [GO:0044470] Sources: GOC:jl